pronephros formation [GO:0072116] (biological process) Also known as: pronephric kidney formation Sources: GOC:mtg_kidney_jan10 Relationships: is a type of animal organ formation [GO:0048645]; is a type of kidney rudiment formation [GO:0072003]; is part of pronephros morphogenesis [GO:0072114] Definition: The developmental process pertaining to the initial formation of the pronephros. In mammals, the pronephros is the first of the three embryonic kidneys to be established and exists only transiently. In lower vertebrates such as fish and amphibia, the pronephros is the fully functional embryonic kidney and is indispensable for larval life. Subtypes: head kidney formation [GO:0072117]